4 iron, 4 sulfur cluster binding [GO:0051539] (molecular function) Also known as: 4 Fe 4 S cluster binding, 4 iron, 4 sulphur cluster binding, 4Fe-4S cluster binding, iron-sulfur cluster 4Fe-4S binding, iron-sulphur cluster 4Fe-4S binding, tetrairon tetrasulfide cluster binding, tetrairon tetrasulphide cluster binding Relationships: is a type of iron-sulfur cluster binding [GO:0051536] Definition: Binding to a 4 iron, 4 sulfur (4Fe-4S) cluster; this cluster consists of four iron atoms, with the inorganic sulfur atoms found between the irons and acting as bridging ligands. References: PMID:15952888 Sources: GOC:ai, Wikipedia:Iron-sulfur_cluster